{
  "term_label": "dynein complex binding",
  "gene": "UniProtKB:Q8N6L0",
  "term_id": "GO:0070840",
  "gene_symbol": "KASH5",
  "gene_name": "Protein KASH5"
}